{
  "gene": "UniProtKB:Q6ZU52",
  "term_label": "Unknown cellular component",
  "gene_symbol": "KIAA0408",
  "gene_name": "Uncharacterized protein KIAA0408",
  "term_id": "UNKNOWN:0003"
}